{
  "term_id": "UNKNOWN:0001",
  "term_label": "Unknown molecular function",
  "gene_symbol": "YLPM1",
  "gene": "UniProtKB:P49750",
  "gene_name": "YLP motif-containing protein 1"
}